{
  "term_label": "Unknown molecular function",
  "term_id": "UNKNOWN:0001",
  "gene_symbol": "ACMSD",
  "gene_name": "2-amino-3-carboxymuconate-6-semialdehyde decarboxylase",
  "gene": "UniProtKB:Q8TDX5"
}